cysteine synthase activity, acting on O-succinyl-L-serine [GO:0141223] (molecular function) Sources: RHEA:53816 Definition: Catalysis of the reaction: hydrogen sulfide + O-succinyl-L-serine = L-cysteine + succinate. Also known as: cysteine synthase activity Relationships: is_a transferase activity, transferring alkyl or aryl (other than methyl) groups [GO:0016765]